regulation of cardiac muscle hypertrophy [GO:0010611] (biological process) Relationships: is a type of GO:0014743; is a type of regulation of muscle adaptation [GO:0043502]; regulates cardiac muscle hypertrophy [GO:0003300] Sources: GOC:dph, GOC:tb Definition: Any process that modulates the rate, frequency or extent of the enlargement or overgrowth of all or part of the heart due to an increase in size (not length) of individual cardiac muscle fibers, without cell division. Subtypes: GO:0010613, GO:0010614, regulation of cardiac muscle hypertrophy in response to stress [GO:1903242]